regulation of natural killer cell mediated cytotoxicity directed against tumor cell target [GO:0002858] (biological process) Relationships: is a type of regulation of natural killer cell mediated immune response to tumor cell [GO:0002855]; is a type of regulation of natural killer cell mediated cytotoxicity [GO:0042269]; RO_0002211 natural killer cell mediated cytotoxicity directed against tumor cell target [GO:0002420] Sources: GOC:add Subtypes: negative regulation of natural killer cell mediated cytotoxicity directed against tumor cell target [GO:0002859], positive regulation of natural killer cell mediated cytotoxicity directed against tumor cell target [GO:0002860] Definition: Any process that modulates the frequency, rate, or extent of natural killer cell mediated cytotoxicity directed against tumor cell target.